{
  "gene_symbol": "PPIP5K2",
  "term_id": "GO:0033857",
  "term_label": "5-diphosphoinositol pentakisphosphate 1-kinase activity",
  "gene": "UniProtKB:O43314",
  "gene_name": "Inositol hexakisphosphate and diphosphoinositol-pentakisphosphate kinase 2"
}